{
  "term_label": "Unknown molecular function",
  "term_id": "UNKNOWN:0001",
  "gene_name": "T cell receptor alpha joining 2 (non-functional) (Fragment)",
  "gene": "UniProtKB:A0A075B6U9",
  "gene_symbol": "TRAJ2"
}